{
  "term_id": "GO:0043524",
  "term_label": "negative regulation of neuron apoptotic process",
  "gene_symbol": "GRINA",
  "gene_name": "Protein lifeguard 1",
  "gene": "UniProtKB:Q7Z429"
}